IgA binding [GO:0019862] (molecular function) Relationships: is a type of immunoglobulin binding [GO:0019865] Definition: Binding to an immunoglobulin of an IgA isotype. Sources: GOC:add, ISBN:0781735149